{
  "gene_name": "Olfactory receptor 8D4",
  "term_label": "odorant binding",
  "gene": "UniProtKB:Q8NGM9",
  "gene_symbol": "OR8D4",
  "term_id": "GO:0005549"
}